{
  "gene_name": "Bleomycin hydrolase",
  "gene_symbol": "BLMH",
  "term_label": "cysteine-type peptidase activity",
  "term_id": "GO:0008234",
  "gene": "UniProtKB:Q13867"
}